{
  "gene_name": "Gamma-aminobutyric acid receptor subunit gamma-2",
  "term_id": "GO:0051932",
  "gene": "UniProtKB:P18507",
  "term_label": "synaptic transmission, GABAergic",
  "gene_symbol": "GABRG2"
}